{
  "gene": "UniProtKB:Q8NCQ7",
  "term_label": "Unknown molecular function",
  "gene_name": "Protein PROCA1",
  "term_id": "UNKNOWN:0001",
  "gene_symbol": "PROCA1"
}